{
  "term_id": "GO:0045202",
  "gene_name": "Dynamin-3",
  "term_label": "synapse",
  "gene_symbol": "DNM3",
  "gene": "UniProtKB:Q9UQ16"
}